{
  "gene_symbol": "VWA5B2",
  "gene_name": "von Willebrand factor A domain-containing protein 5B2",
  "term_label": "Unknown biological process",
  "term_id": "UNKNOWN:0002",
  "gene": "UniProtKB:Q8N398"
}